{
  "term_id": "GO:0007288",
  "gene": "UniProtKB:Q6ZU64",
  "term_label": "sperm axoneme assembly",
  "gene_symbol": "CFAP65",
  "gene_name": "Cilia- and flagella-associated protein 65"
}